{
  "gene": "UniProtKB:Q9H354",
  "gene_symbol": "PRO1933",
  "term_label": "Unknown biological process",
  "gene_name": "Putative uncharacterized protein PRO1933",
  "term_id": "UNKNOWN:0002"
}